{
  "gene_name": "Spliceosome RNA helicase DDX39B",
  "term_id": "UNKNOWN:0003",
  "term_label": "Unknown cellular component",
  "gene_symbol": "DDX39B",
  "gene": "UniProtKB:Q13838"
}